{
  "term_label": "DNA topoisomerase III-beta-TDRD3 complex",
  "gene": "UniProtKB:Q9H7E2",
  "gene_name": "Tudor domain-containing protein 3",
  "gene_symbol": "TDRD3",
  "term_id": "GO:0140225"
}